{
  "gene": "UniProtKB:P62699",
  "gene_name": "Protein yippee-like 5",
  "term_label": "ubiquitin ligase complex",
  "gene_symbol": "YPEL5",
  "term_id": "GO:0000151"
}